L-diaminopimelate transmembrane transporter activity [GO:0015626] (molecular function) Definition: Enables the transfer of L-diaminopimelate from one side of a membrane to the other. L-diaminopimelate is the L-enantiomer anion of 2,6-diaminoheptanedioic acid. Relationships: is a type of GO:0015179; is part of diaminopimelate transport [GO:0015830] Also known as: L-diaminopimelate transporter activity, cystine/diaminopimelate porter activity Sources: GOC:go_curators, GOC:jsg, GOC:mah, GOC:mtg_transport, ISBN:0198506732